{
  "term_label": "Unknown biological process",
  "gene_symbol": "Q6ZRU5",
  "gene": "UniProtKB:Q6ZRU5",
  "gene_name": "Putative uncharacterized protein FLJ46089",
  "term_id": "UNKNOWN:0002"
}